large latent transforming growth factor-beta complex [GO:0038045] (cellular component) Relationships: is a type of protein-containing complex [GO:0032991] Also known as: LLC, large latent complex References: PMID:2350783, PMID:8680476, PMID:9805445 Sources: GOC:bf Definition: A protein complex containing latency-associated proteins (LAPs), mature disulphide-linked dimeric TGF-beta, and latent TGF-beta binding proteins (LTBPs). TGF-beta is mostly secreted as part of the large latent complex, and must be subsequently released from the LLC in order to bind to cell surface receptors.